{
  "term_label": "ATPase activator activity",
  "term_id": "GO:0001671",
  "gene_symbol": "DNAJA1",
  "gene": "UniProtKB:P31689",
  "gene_name": "DnaJ homolog subfamily A member 1"
}